{
  "term_label": "small GTPase binding",
  "term_id": "GO:0031267",
  "gene": "UniProtKB:Q14161",
  "gene_name": "ARF GTPase-activating protein GIT2",
  "gene_symbol": "GIT2"
}